{
  "term_label": "Unknown cellular component",
  "gene_name": "Dynein axonemal light chain 4",
  "gene": "UniProtKB:O96015",
  "gene_symbol": "DNAL4",
  "term_id": "UNKNOWN:0003"
}